{
  "term_label": "cytosolic large ribosomal subunit",
  "gene_name": "Large ribosomal subunit protein uL24",
  "gene": "UniProtKB:P61254",
  "gene_symbol": "RPL26",
  "term_id": "GO:0022625"
}